insulin secretion [GO:0030073] (biological process) Subtypes: insulin secretion involved in cellular response to glucose stimulus [GO:0035773] Relationships: is a type of protein secretion [GO:0009306]; is a type of peptide hormone secretion [GO:0030072] Sources: GOC:mah, ISBN:0198506732 Regulation: positively regulated by positive regulation of insulin secretion [GO:0032024]; negatively regulated by negative regulation of insulin secretion [GO:0046676]; regulated by regulation of insulin secretion [GO:0050796] Definition: The regulated release of proinsulin from secretory granules accompanied by cleavage of proinsulin to form mature insulin. In vertebrates, insulin is secreted from B granules in the B cells of the vertebrate pancreas and from insulin-producing cells in insects.